{
  "gene_name": "Polyglutamylase complex subunit TTLL1",
  "gene_symbol": "TTLL1",
  "term_label": "tubulin-glutamic acid ligase activity",
  "term_id": "GO:0070740",
  "gene": "UniProtKB:O95922"
}